{
  "gene_name": "Ubiquitin carboxyl-terminal hydrolase 17",
  "gene": "UniProtKB:Q6R6M4",
  "term_id": "GO:0004843",
  "term_label": "cysteine-type deubiquitinase activity",
  "gene_symbol": "USP17L2"
}